{
  "gene_symbol": "PKIG",
  "term_id": "GO:0005634",
  "gene_name": "cAMP-dependent protein kinase inhibitor gamma",
  "gene": "UniProtKB:Q9Y2B9",
  "term_label": "nucleus"
}